{
  "term_label": "Unknown molecular function",
  "gene_name": "LHFPL tetraspan subfamily member 3 protein",
  "term_id": "UNKNOWN:0001",
  "gene": "UniProtKB:Q86UP9",
  "gene_symbol": "LHFPL3"
}